{
  "term_label": "Unknown cellular component",
  "term_id": "UNKNOWN:0003",
  "gene": "UniProtKB:P09238",
  "gene_symbol": "MMP10",
  "gene_name": "Stromelysin-2"
}